{
  "term_id": "GO:0003899",
  "term_label": "DNA-directed RNA polymerase activity",
  "gene_name": "DNA-directed RNA polymerase II subunit RPB9",
  "gene": "UniProtKB:P36954",
  "gene_symbol": "POLR2I"
}